{
  "gene_name": "Adhesion G protein-coupled receptor B3",
  "term_id": "GO:0005886",
  "gene_symbol": "ADGRB3",
  "gene": "UniProtKB:O60242",
  "term_label": "plasma membrane"
}